{
  "gene_name": "Solute carrier family 15 member 1",
  "term_id": "GO:0005886",
  "gene_symbol": "SLC15A1",
  "term_label": "plasma membrane",
  "gene": "UniProtKB:P46059"
}